negative regulation of Rho-dependent protein serine/threonine kinase activity [GO:2000299] (biological process) Definition: Any process that stops, prevents or reduces the frequency, rate or extent of Rho-dependent protein serine/threonine kinase activity. Relationships: is a type of negative regulation of protein serine/threonine kinase activity [GO:0071901]; is a type of regulation of Rho-dependent protein serine/threonine kinase activity [GO:2000298]; negatively regulates Rho-dependent protein serine/threonine kinase activity [GO:0072518] Sources: GOC:mah Also known as: negative regulation of ROCK kinase activity, negative regulation of Rho-associated protein kinase activity